{
  "term_label": "endocytosis",
  "gene": "UniProtKB:Q9UL26",
  "gene_symbol": "RAB22A",
  "term_id": "GO:0006897",
  "gene_name": "Ras-related protein Rab-22A"
}